UDP-xylose transmembrane transporter activity [GO:0005464] (MF) Relationships: is a type of pyrimidine nucleotide-sugar transmembrane transporter activity [GO:0015165]; is part of UDP-xylose transmembrane transport [GO:0015790] Definition: Enables the transfer of UDP-xylose from one side of a membrane to the other. UDP-xylose is a substance composed of xylose in glycosidic linkage with uridine diphosphate. Sources: GOC:ai